{
  "gene": "UniProtKB:A9Z1Z3",
  "gene_symbol": "FER1L4",
  "gene_name": "Fer-1-like protein 4",
  "term_label": "Unknown molecular function",
  "term_id": "UNKNOWN:0001"
}